{
  "term_label": "Unknown molecular function",
  "term_id": "UNKNOWN:0001",
  "gene": "UniProtKB:Q13015",
  "gene_symbol": "MLLT11",
  "gene_name": "Protein AF1q"
}